{
  "term_label": "Unknown molecular function",
  "gene": "UniProtKB:Q5THR3",
  "gene_symbol": "EFCAB6",
  "gene_name": "EF-hand calcium-binding domain-containing protein 6",
  "term_id": "UNKNOWN:0001"
}